{
  "gene_symbol": "CPT1B",
  "term_id": "GO:0005739",
  "term_label": "mitochondrion",
  "gene_name": "Carnitine O-palmitoyltransferase 1, muscle isoform",
  "gene": "UniProtKB:Q92523"
}